photosystem II reaction center [GO:0009539] (cellular component) Also known as: photosystem II reaction centre Definition: An integral membrane complex containing P680, the chlorophyll a molecule that functions as a primary electron donor. In the light, functioning as a water-plastoquinone oxidoreductase, it transfers electrons from water to plastoquinone. Sources: GOC:kd, ISBN:0943088399 Relationships: is a type of membrane protein complex [GO:0098796]; is part of photosystem II [GO:0009523]